{
  "gene": "UniProtKB:Q7Z6Z7",
  "gene_name": "E3 ubiquitin-protein ligase HUWE1",
  "term_id": "GO:0005737",
  "term_label": "cytoplasm",
  "gene_symbol": "HUWE1"
}